{
  "term_id": "GO:0030016",
  "gene_name": "Leiomodin-1",
  "term_label": "myofibril",
  "gene": "UniProtKB:P29536",
  "gene_symbol": "LMOD1"
}